{
  "gene_name": "GDP-fucose protein O-fucosyltransferase 1",
  "term_label": "endoplasmic reticulum",
  "term_id": "GO:0005783",
  "gene_symbol": "POFUT1",
  "gene": "UniProtKB:Q9H488"
}